protein-arginine N-methyltransferase activity [GO:0016274] (molecular function) Relationships: is a type of protein methyltransferase activity [GO:0008276]; is a type of arginine N-methyltransferase activity [GO:0016273] Also known as: PRMT activity Definition: Catalysis of the reaction: S-adenosyl-L-methionine + (protein)-arginine = S-adenosyl-L-homocysteine + (protein)-N-methyl-arginine. References: PMID:12351636, PMID:31284549 Sources: GOC:mah Subtypes: protein arginine N5-methyltransferase activity [GO:0019702], protein-arginine omega-N monomethyltransferase activity [GO:0035241], protein-arginine omega-N asymmetric methyltransferase activity [GO:0035242], protein-arginine omega-N symmetric methyltransferase activity [GO:0035243], histone H3R17 methyltransferase activity [GO:0035642], histone H4R3 methyltransferase activity [GO:0044020], histone H3R2 methyltransferase activity [GO:0070611], GO:0070612, GO:0140592, histone H3R26 methyltransferase activity [GO:0140903]